dendritic transport [GO:0098935] (biological process) Subtypes: retrograde dendritic transport [GO:0098934], anterograde dendritic transport [GO:0098937], dendritic transport of mitochondrion [GO:0098939], dendritic transport of ribonucleoprotein complex [GO:0098961], dendritic transport of messenger ribonucleoprotein complex [GO:0098963] Definition: The directed movement of organelles or molecules along microtubules in dendrites. Also known as: dendrite cargo transport Relationships: is a type of GO:0008088; BFO_0000066 dendrite [GO:0030425] Sources: ISBN:0815316194